{
  "term_id": "GO:0000981",
  "gene": "UniProtKB:Q8NF99",
  "gene_symbol": "ZNF397",
  "gene_name": "Zinc finger protein 397",
  "term_label": "DNA-binding transcription factor activity, RNA polymerase II-specific"
}